positive regulation of retrograde axon cargo transport [GO:2001019] (biological process) Definition: Any process that activates or increases the frequency, rate or extent of retrograde axon cargo transport. Relationships: is a type of GO:0032388; is_a regulation of retrograde axon cargo transport [GO:2001017]; positively regulates retrograde axonal transport [GO:0008090] Also known as: positive regulation of retrograde axonal transport Sources: GOC:obol Subtypes: positive regulation of retrograde dense core granule transport [GO:1901956]